{
  "gene_symbol": "CDH4",
  "term_id": "GO:0008013",
  "term_label": "beta-catenin binding",
  "gene": "UniProtKB:P55283",
  "gene_name": "Cadherin-4"
}